{
  "gene_symbol": "TNIP1",
  "gene": "UniProtKB:Q15025",
  "term_id": "GO:0006357",
  "term_label": "regulation of transcription by RNA polymerase II",
  "gene_name": "TNFAIP3-interacting protein 1"
}